{
  "term_label": "actin filament",
  "term_id": "GO:0005884",
  "gene": "UniProtKB:P60709",
  "gene_symbol": "ACTB",
  "gene_name": "Actin, cytoplasmic 1"
}